{
  "term_id": "GO:0045944",
  "term_label": "positive regulation of transcription by RNA polymerase II",
  "gene_symbol": "SMAD2",
  "gene": "UniProtKB:Q15796",
  "gene_name": "Mothers against decapentaplegic homolog 2"
}